suppression of viral release by host [GO:0044790] (biological process) References: PMID:18305167 Sources: GOC:jl Relationships: is a type of defense response to virus [GO:0051607] Also known as: down regulation of release of virus from host, down regulation of viral exit, down regulation of viral release, down regulation of viral release from host cell, down regulation of viral shedding, down-regulation of release of virus from host, down-regulation of viral exit, down-regulation of viral release, down-regulation of viral release from host cell, down-regulation of viral shedding, downregulation of release of virus from host, downregulation of viral exit, downregulation of viral release, downregulation of viral release from host cell, downregulation of viral shedding, inhibition of release of virus from host, inhibition of viral exit, inhibition of viral release, inhibition of viral shedding, negative regulation by host of viral release from host cell, negative regulation of release of virus from host, negative regulation of viral exit, negative regulation of viral release, negative regulation of viral release from host cell, negative regulation of viral shedding, inhibition of viral release from host cell Definition: A process in which a host organism stops, prevents or reduces the frequency, rate or extent of the release of a virus with which it is infected, from its cells.